{
  "gene_name": "Rho guanine nucleotide exchange factor 12",
  "term_label": "guanyl-nucleotide exchange factor activity",
  "term_id": "GO:0005085",
  "gene_symbol": "ARHGEF12",
  "gene": "UniProtKB:Q9NZN5"
}